protein-N-terminal-alanine acetyltransferase activity [GO:0008999] (molecular function) Sources: RHEA:50500 Also known as: ribosomal-protein-alanine N-acetyltransferase activity, peptide-alanine-alpha-N-acetyltransferase activity, acetyl-CoA:ribosomal-protein-L-alanine N-acetyltransferase activity, ribosomal protein S18 acetyltransferase activity Relationships: is a type of protein-N-terminal amino-acid acetyltransferase activity [GO:0004596] Definition: Catalysis of the reaction: acetyl-CoA + N-terminal L-alanyl-[protein] = CoA + H+ + N-terminal N(alpha)-acetyl-L-alanyl-[protein].